{
  "gene": "UniProtKB:Q7Z7G0",
  "gene_symbol": "ABI3BP",
  "term_id": "UNKNOWN:0002",
  "gene_name": "Target of Nesh-SH3",
  "term_label": "Unknown biological process"
}